positive regulation of type B pancreatic cell proliferation [GO:1904692] (biological process) Also known as: positive regulation of pancreatic B cell proliferation, positive regulation of pancreatic beta cell proliferation, up regulation of pancreatic B cell proliferation, up regulation of pancreatic beta cell proliferation, up regulation of type B pancreatic cell proliferation, up-regulation of pancreatic B cell proliferation, up-regulation of pancreatic beta cell proliferation, up-regulation of type B pancreatic cell proliferation, upregulation of pancreatic B cell proliferation, upregulation of pancreatic beta cell proliferation, upregulation of type B pancreatic cell proliferation, activation of pancreatic B cell proliferation, activation of pancreatic beta cell proliferation, activation of type B pancreatic cell proliferation References: PMID:24055447 Sources: GOC:TermGenie, GO_REF:0000058 Definition: Any process that activates or increases the frequency, rate or extent of type B pancreatic cell proliferation. Relationships: is a type of positive regulation of epithelial cell proliferation [GO:0050679]; is_a GO:0061469; positively regulates type B pancreatic cell proliferation [GO:0044342]